{
  "term_label": "anterior/posterior pattern specification",
  "gene": "UniProtKB:Q9C0J9",
  "gene_symbol": "BHLHE41",
  "gene_name": "Class E basic helix-loop-helix protein 41",
  "term_id": "GO:0009952"
}